{
  "gene_symbol": "ERCC4",
  "term_label": "nucleotide-excision repair involved in interstrand cross-link repair",
  "gene": "UniProtKB:Q92889",
  "gene_name": "DNA repair endonuclease XPF",
  "term_id": "GO:1901255"
}